{
  "gene": "UniProtKB:Q9H9Q2",
  "gene_symbol": "COPS7B",
  "term_label": "Unknown molecular function",
  "term_id": "UNKNOWN:0001",
  "gene_name": "COP9 signalosome complex subunit 7b"
}